{
  "gene_name": "Cytoplasmic polyadenylation element-binding protein 3",
  "term_id": "GO:0045202",
  "gene_symbol": "CPEB3",
  "term_label": "synapse",
  "gene": "UniProtKB:Q8NE35"
}